schizogony [GO:0020014] (biological process) Definition: Cell division by multiple fission in which nuclei and other organelles in the parent cell divide repeatedly and move to the cell periphery before internal membranes develop around them, producing a large number of daughter cells simultaneously. Sources: GOC:mb Relationships: is a type of cell division [GO:0051301]